positive regulation of secondary heart field cardioblast proliferation [GO:0072513] (biological process) Definition: Any process that activates or increases the frequency, rate or extent of cardioblast proliferation in the second heart field. A cardioblast is a cardiac precursor cell. It is a cell that has been committed to a cardiac fate, but will undergo more cell division rather than terminally differentiating. The secondary heart field is the region of the heart that will form the majority of the mesodermal component of the right ventricle, the arterial pole (outflow tract) and the venous pole (inflow tract). Sources: GOC:BHF, GOC:mah, GOC:rl Relationships: is a type of regulation of secondary heart field cardioblast proliferation [GO:0003266]; is a type of positive regulation of cell population proliferation [GO:0008284] Also known as: negative regulation of second heart field cardioblast proliferation